{
  "gene_symbol": "MARCHF1",
  "gene": "UniProtKB:Q8TCQ1",
  "gene_name": "E3 ubiquitin-protein ligase MARCHF1",
  "term_id": "GO:0005764",
  "term_label": "lysosome"
}